{
  "gene_symbol": "ANGEL1",
  "term_label": "mRNA 3'-UTR binding",
  "gene_name": "Protein angel homolog 1",
  "gene": "UniProtKB:Q9UNK9",
  "term_id": "GO:0003730"
}